{
  "term_label": "Unknown biological process",
  "gene_name": "Ovochymase-2",
  "gene_symbol": "OVCH2",
  "term_id": "UNKNOWN:0002",
  "gene": "UniProtKB:Q7RTZ1"
}